{
  "term_label": "innate immune response",
  "gene": "UniProtKB:Q8IUB2",
  "gene_name": "WAP four-disulfide core domain protein 3",
  "term_id": "GO:0045087",
  "gene_symbol": "WFDC3"
}